{
  "gene_name": "Tetratricopeptide repeat protein 39B",
  "term_id": "GO:0042632",
  "gene_symbol": "TTC39B",
  "term_label": "cholesterol homeostasis",
  "gene": "UniProtKB:Q5VTQ0"
}